{
  "term_label": "nucleus",
  "term_id": "GO:0005634",
  "gene_symbol": "TBRG1",
  "gene_name": "Transforming growth factor beta regulator 1",
  "gene": "UniProtKB:Q3YBR2"
}